regulation of blood volume by renin-angiotensin [GO:0002016] (biological process) Sources: GOC:dph, GOC:mtg_cardio, GOC:tb, ISBN:0721643949 Definition: The process in which the renin-angiotensin system controls the rate of fluid intake and output into the blood. Relationships: is a type of regulation of systemic arterial blood pressure by renin-angiotensin [GO:0003081] Also known as: renin-angiotensin regulation of blood volume, renin-angiotensin control of body fluid levels Subtypes: regulation of renal output by angiotensin [GO:0002019], brain renin-angiotensin system [GO:0002035]